negative regulation of B cell activation [GO:0050869] (biological process) Relationships: is a type of GO:0050864; is_a GO:0051250; negatively regulates B cell activation [GO:0042113] Sources: GOC:ai Definition: Any process that stops, prevents, or reduces the frequency, rate or extent of B cell activation. Subtypes: GO:0030889, negative regulation of B cell differentiation [GO:0045578], negative regulation of isotype switching [GO:0045829] Also known as: down regulation of B cell activation, down-regulation of B cell activation, downregulation of B cell activation, negative regulation of B lymphocyte activation, negative regulation of B-cell activation, negative regulation of B-lymphocyte activation, inhibition of B cell activation